{
  "term_id": "GO:0031267",
  "gene": "UniProtKB:Q9H2M9",
  "gene_symbol": "RAB3GAP2",
  "gene_name": "Rab3 GTPase-activating protein non-catalytic subunit",
  "term_label": "small GTPase binding"
}